{
  "gene_symbol": "GTF3C6",
  "gene": "UniProtKB:Q969F1",
  "gene_name": "General transcription factor 3C polypeptide 6",
  "term_id": "GO:0006383",
  "term_label": "transcription by RNA polymerase III"
}